{
  "gene": "UniProtKB:P00742",
  "term_label": "blood coagulation",
  "gene_symbol": "F10",
  "term_id": "GO:0007596",
  "gene_name": "Coagulation factor X"
}